{
  "gene_symbol": "WASHC5",
  "gene": "UniProtKB:Q12768",
  "gene_name": "WASH complex subunit 5",
  "term_id": "GO:0071203",
  "term_label": "WASH complex"
}